{
  "term_label": "Unknown cellular component",
  "term_id": "UNKNOWN:0003",
  "gene_name": "Overexpressed in colon carcinoma 1 protein",
  "gene_symbol": "OCC1",
  "gene": "UniProtKB:Q8TAD7"
}